{
  "gene": "UniProtKB:Q96RP3",
  "gene_name": "Urocortin-2",
  "gene_symbol": "UCN2",
  "term_id": "GO:0009755",
  "term_label": "hormone-mediated signaling pathway"
}